3-hydroxycyclohexanone dehydrogenase activity [GO:0047564] (molecular function) Relationships: is a type of oxidoreductase activity, acting on CH-OH group of donors [GO:0016614] Sources: EC:1.1.99.26, RHEA:15905 Definition: Catalysis of the reaction: 3-hydroxycyclohexanone + A = AH(2) + cyclohexane-1,3-dione. Also known as: 3-hydroxycyclohexanone:acceptor 1-oxidoreductase activity